{
  "term_id": "UNKNOWN:0001",
  "term_label": "Unknown molecular function",
  "gene_name": "Suppressor of tumorigenicity 7 protein-like",
  "gene": "UniProtKB:Q8TDW4",
  "gene_symbol": "ST7L"
}